{
  "term_id": "GO:0005776",
  "gene_name": "Autophagy-related protein 13",
  "gene_symbol": "ATG13",
  "term_label": "autophagosome",
  "gene": "UniProtKB:O75143"
}